innate immune response-activating signaling pathway [GO:0002758] (biological process) Also known as: effector triggered immunity, effector-triggered immunity, defence response signaling pathway, resistance gene-dependent, defence response signaling pathway, resistance gene-independent, defence response signalling pathway, resistance gene-dependent, defence response signalling pathway, resistance gene-independent, defense response signaling pathway, resistance gene-dependent, defense response signaling pathway, resistance gene-independent, defense response signalling pathway, resistance gene-dependent, effector-triggered immune signaling Subtypes: innate immune response activating cell surface receptor signaling pathway [GO:0002220], pattern recognition receptor signaling pathway [GO:0002221] References: PMID:11418339, PMID:28105028 Sources: GOC:jy, GOC:mah Relationships: is a type of activation of innate immune response [GO:0002218]; is a type of immune response-activating signaling pathway [GO:0002757] Definition: The series of molecular signals generated by a ligand binding to its receptor that lead to the activation or perpetuation of an innate immune response.